{
  "gene_name": "Podoplanin",
  "term_label": "Unknown molecular function",
  "gene": "UniProtKB:Q86YL7",
  "gene_symbol": "PDPN",
  "term_id": "UNKNOWN:0001"
}